{
  "gene_name": "Mitochondrial carrier homolog 2",
  "term_id": "GO:0016020",
  "term_label": "membrane",
  "gene_symbol": "MTCH2",
  "gene": "UniProtKB:Q9Y6C9"
}